skeletal muscle cell differentiation [GO:0035914] (BP) Definition: The process in which a relatively unspecialized cell acquires specialized features of a skeletal muscle cell, a somatic cell located in skeletal muscle. Relationships: is a type of cell differentiation [GO:0030154]; is part of skeletal muscle tissue development [GO:0007519] Subtypes: skeletal muscle satellite cell differentiation [GO:0014816], GO:0098528 Regulation: RO_0002211 by regulation of skeletal muscle cell differentiation [GO:2001014]; negatively regulated by negative regulation of skeletal muscle cell differentiation [GO:2001015]; positively regulated by positive regulation of skeletal muscle cell differentiation [GO:2001016] Sources: CL:0000188, GOC:BHF, GOC:vk